{
  "gene_name": "Syndecan-1",
  "term_id": "UNKNOWN:0001",
  "gene": "UniProtKB:P18827",
  "term_label": "Unknown molecular function",
  "gene_symbol": "SDC1"
}